{
  "gene_name": "Islet cell autoantigen 1",
  "term_id": "GO:0097753",
  "gene": "UniProtKB:Q05084",
  "gene_symbol": "ICA1",
  "term_label": "membrane bending"
}